{
  "gene_name": "Hsp90 co-chaperone Cdc37-like 1",
  "term_id": "GO:0050821",
  "gene_symbol": "CDC37L1",
  "gene": "UniProtKB:Q7L3B6",
  "term_label": "protein stabilization"
}